{
  "gene_name": "Unconventional myosin-IXb",
  "gene_symbol": "MYO9B",
  "gene": "UniProtKB:Q13459",
  "term_label": "ATP hydrolysis activity",
  "term_id": "GO:0016887"
}